2,4-dihydroxy-7-methoxy-2H-1,4-benzoxazin-3(4H)-one 2-D-glucosyltransferase activity [GO:0047254] (molecular function) Also known as: UDP-glucose:2,4-dihydroxy-7-methoxy-2H-1,4-benzoxazin-3(4H)-one 2-D-glucosyltransferase activity, UDPglucose:2,4-dihydroxy-7-methoxy-2H-1,4-benzoxazin-3(4H)-one 2-D-glucosyltransferase activity, uridine diphosphoglucose-2,4-dihydroxy-7-methoxy-2H-1,4-benzoxazin-3(4H)-one 2-glucosyltransferase activity Definition: Catalysis of the reaction: 2,4-dihydroxy-7-methoxy-2H-1,4-benzoxazin-3(4H)-one + UDP-D-glucose = 2,4-dihydroxy-7-methoxy-2H-1,4-benzoxazin-3(4H)-one 2-D-glucoside + UDP. Sources: EC:2.4.1.202 Relationships: is a type of GO:0035251